regulation of leukocyte migration [GO:0002685] (biological process) Also known as: regulation of immune cell migration, regulation of leucocyte migration Definition: Any process that modulates the frequency, rate, or extent of leukocyte migration. Relationships: is a type of regulation of immune system process [GO:0002682]; is_a regulation of cell migration [GO:0030334]; regulates GO:0050900 Sources: GOC:add Subtypes: GO:0002686, positive regulation of leukocyte migration [GO:0002687], regulation of leukocyte chemotaxis [GO:0002688], regulation of cellular extravasation [GO:0002691], regulation of mononuclear cell migration [GO:0071675], regulation of neutrophil migration [GO:1902622], regulation of eosinophil migration [GO:2000416]